{
  "term_id": "GO:0009952",
  "term_label": "anterior/posterior pattern specification",
  "gene_symbol": "HOXC6",
  "gene": "UniProtKB:P09630",
  "gene_name": "Homeobox protein Hox-C6"
}